{
  "gene": "UniProtKB:P0C879",
  "gene_symbol": "P0C879",
  "gene_name": "Putative uncharacterized protein FLJ43185",
  "term_id": "UNKNOWN:0003",
  "term_label": "Unknown cellular component"
}